{
  "term_label": "Unknown cellular component",
  "term_id": "UNKNOWN:0003",
  "gene_symbol": "AMDHD1",
  "gene": "UniProtKB:Q96NU7",
  "gene_name": "Probable imidazolonepropionase"
}